L-homomethionine biosynthetic process [GO:0033322] (biological process) Definition: The chemical reactions and pathways resulting in the formation of L-homomethionine, a non-protein amino acid synthesized from L-methionine via chain elongation. Relationships: is a type of carboxylic acid biosynthetic process [GO:0046394] Sources: GOC:mah, MetaCyc:PWY-1186 Also known as: homomethionine anabolism, homomethionine biosynthesis, homomethionine biosynthetic process, homomethionine formation, homomethionine synthesis